P-type calcium transporter activity involved in regulation of cardiac muscle cell membrane potential [GO:0086039] (molecular function) Definition: A calcium-transporting P-type ATPase activity involved in regulation of the plasma membrane potential. Sources: GOC:BHF, GOC:mtg_cardiac_conduct_nov11 Relationships: is_a P-type calcium transporter activity [GO:0005388]; is part of regulation of cardiac muscle cell membrane potential [GO:0086036] Also known as: calcium-transporting ATPase activity involved in regulation of cardiac muscle cell membrane potential